mitochondrial RNA 3'-end processing [GO:0000965] (biological process) Definition: Any process involved in forming the mature 3' end of an RNA molecule transcribed from a mitochondrial genome; occurs in the mitochondrion. Relationships: is a type of mitochondrial RNA processing [GO:0000963]; is a type of RNA 3'-end processing [GO:0031123] Also known as: mitochondrial RNA 3' end processing Subtypes: mitochondrial mRNA 3'-end processing [GO:0090616], mitochondrial tRNA 3'-end processing [GO:1990180] Sources: GOC:krc, GOC:mah